nicotianamine synthase activity [GO:0030410] (molecular function) Definition: Catalysis of the reaction: 3 S-adenosyl-L-methionine(1+) = 3 S-methyl-5'-thioadenosine + 3 H+ + nicotianamine. Sources: EC:2.5.1.43, RHEA:16481 Also known as: S-adenosyl-L-methionine:S-adenosyl-L-methionine:S-adenosyl-L-methionine 3-amino-3-carboxypropyltransferase activity Relationships: is a type of transferase activity, transferring alkyl or aryl (other than methyl) groups [GO:0016765]